{
  "gene_symbol": "FOXC2",
  "term_id": "GO:0000978",
  "gene": "UniProtKB:Q99958",
  "term_label": "RNA polymerase II cis-regulatory region sequence-specific DNA binding",
  "gene_name": "Forkhead box protein C2"
}